positive regulation of tolerance induction dependent upon immune response [GO:0002654] (biological process) Subtypes: positive regulation of tolerance induction to nonself antigen [GO:0002657], positive regulation of peripheral tolerance induction [GO:0002660] Also known as: positive regulation of immune response-dependent tolerance induction, up regulation of tolerance induction dependent upon immune response, up-regulation of tolerance induction dependent upon immune response, upregulation of tolerance induction dependent upon immune response, activation of tolerance induction dependent upon immune response, stimulation of tolerance induction dependent upon immune response Definition: Any process that activates or increases the frequency, rate, or extent of tolerance induction dependent upon immune response. Sources: GOC:add Relationships: is a type of GO:0002645; is a type of regulation of tolerance induction dependent upon immune response [GO:0002652]; is a type of GO:0002824; positively regulates tolerance induction dependent upon immune response [GO:0002461]